regulation of mitotic nuclear envelope disassembly [GO:1905557] (biological process) Relationships: is a type of regulation of membrane disassembly [GO:0010549]; is a type of regulation of cell cycle process [GO:0010564]; regulates GO:0007077 Subtypes: GO:1905558, positive regulation of mitotic nuclear envelope disassembly [GO:1905559] References: PMID:18765790 Sources: GOC:TermGenie, GO_REF:0000058 Also known as: regulation of mitotic nuclear envelope breakdown, regulation of mitotic nuclear envelope catabolism, regulation of mitotic nuclear envelope degradation Definition: Any process that modulates the frequency, rate or extent of mitotic nuclear envelope disassembly.